gamma-tubulin complex assembly [GO:1902481] (biological process) Definition: The aggregation, arrangement and bonding together of a set of components to form a gamma-tubulin complex. References: PMID:23885124 Sources: GOC:TermGenie Also known as: gamma-tubulin complex formation Relationships: is a type of protein-containing complex assembly [GO:0065003]